cellular response to calcium ion [GO:0071277] (biological process) Sources: GOC:mah Also known as: cellular response to Ca2+ ion Relationships: is a type of response to calcium ion [GO:0051592]; is a type of cellular response to metal ion [GO:0071248] Definition: Any process that results in a change in state or activity of a cell (in terms of movement, secretion, enzyme production, gene expression, etc.) as a result of a calcium ion stimulus.